plasma membrane invagination [GO:0099024] (biological process) Sources: GOC:dos, GOC:vw Subtypes: phagocytosis, engulfment [GO:0006911], GO:0036089, cleavage furrow ingression [GO:0036090] Relationships: is a type of membrane invagination [GO:0010324] Definition: An infolding of the plasma membrane.